fatty acid primary amide catabolic process [GO:0062127] (biological process) Definition: The chemical reactions and pathways resulting in the breakdown of primary fatty amides. Relationships: is a type of GO:0062126; is a type of fatty acid derivative catabolic process [GO:1901569] Also known as: primary fatty amide catabolic process References: PMID:11128635